synaptotagmin-synaptobrevin 2-SNAP-25-syntaxin-1a-syntaxin-1b-Rab3a complex [GO:0070356] (cellular component) Definition: A SNARE complex that contains synaptotagmin, synaptobrevin 2 (VAMP2), SNAP-25, syntaxin 1a, syntaxin1b, and Rab3a (or orthologs thereof). References: PMID:7654227 Also known as: SNARE complex (STX1a, STX1b, SNAP25, RAB3a, SYT1, VAMP2), STX1a-STX1b-SNAP25-RAB3a-SYT1-VAMP2 complex Relationships: is_a SNARE complex [GO:0031201]